retrotransposon nucleocapsid [GO:0000943] (cellular component) Definition: A complex of the retrotransposon RNA genome, reverse transcriptase, integrase, and associated molecules required for reproduction and integration of the retrotransposon into the host genome; the main structural molecule of the nucleocapsid is often a gag protein homolog. References: PMID:10861903 Sources: GOC:clt Relationships: is a type of cellular anatomical structure [GO:0110165]; is part of nucleus [GO:0005634] Also known as: VLP, Virus-like particle